{
  "gene": "UniProtKB:Q53EV4",
  "gene_name": "Leucine-rich repeat-containing protein 23",
  "term_label": "Unknown molecular function",
  "gene_symbol": "LRRC23",
  "term_id": "UNKNOWN:0001"
}